{
  "gene_symbol": "MAB21L3",
  "term_id": "UNKNOWN:0002",
  "term_label": "Unknown biological process",
  "gene": "UniProtKB:Q8N8X9",
  "gene_name": "Protein mab-21-like 3"
}